type III site-specific deoxyribonuclease complex [GO:0019813] (cellular component) Definition: A heterodimeric enzyme complex composed of two subunits, Res and Mod, that functions as an endonuclease and cleaves DNA. Cleavage will only occur when there are two un-methylated copies of a specific recognition site in an inverse orientation on the DNA. Cleavage occurs at a specific distance away from one of the recognition sites. The Mod subunit can act alone as a methyltansferase. DNA restriction systems such as this are used by bacteria to defend against phage and other foreign DNA that may enter a cell. References: PMID:12654995 Also known as: type III restriction enzyme complex Relationships: is a type of endodeoxyribonuclease complex [GO:1905347]; is part of cytoplasm [GO:0005737]